{
  "gene_symbol": "PIK3C2G",
  "term_id": "GO:0048015",
  "gene_name": "Phosphatidylinositol 3-kinase C2 domain-containing subunit gamma",
  "term_label": "phosphatidylinositol-mediated signaling",
  "gene": "UniProtKB:O75747"
}